{
  "term_label": "circadian regulation of gene expression",
  "gene_name": "Nuclear receptor-interacting protein 1",
  "gene_symbol": "NRIP1",
  "gene": "UniProtKB:P48552",
  "term_id": "GO:0032922"
}